purine ribonucleotide salvage [GO:0106380] (biological process) Relationships: is a type of purine ribonucleotide biosynthetic process [GO:0009152]; is a type of purine nucleotide salvage [GO:0032261] Definition: Any process which produces a purine ribonucleotide from derivatives of it, without de novo synthesis. References: PMID:8864750 Subtypes: GMP salvage [GO:0032263], IMP salvage [GO:0032264], XMP salvage [GO:0032265], AMP salvage [GO:0044209]